positive regulation of the force of heart contraction [GO:0098735] (biological process) References: PMID:17242280 Sources: GOC:BHF, GOC:dos, GOC:mtg_cardiac_conduct_nov11, GOC:rl Definition: Any process that increases the force of heart muscle contraction. Relationships: is a type of regulation of the force of heart contraction [GO:0002026]